{
  "gene_name": "TNFAIP3-interacting protein 2",
  "gene_symbol": "TNIP2",
  "gene": "UniProtKB:Q8NFZ5",
  "term_id": "GO:0006357",
  "term_label": "regulation of transcription by RNA polymerase II"
}